9+0 motile cilium [GO:0097728] (cellular component) Relationships: is a type of motile cilium [GO:0031514]; has part inner dynein arm [GO:0036156]; has part outer dynein arm [GO:0036157]; has part axonemal doublet microtubule [GO:0097545] Definition: A motile cilium where the axoneme has a ring of nine outer microtubule doublets but no central microtubules (and is therefore called a 9+0 axoneme). Note: This type of cilia may be present in solitary (classic nodal cilia in embryonic nodes) or in multiple copies (e.g. in the choroid plexus epithelium). Also known as: motile 9+0 cilium, nodal cilium References: PMID:10330409, PMID:22118931 Sources: GOC:cilia